{
  "gene_symbol": "SCARB2",
  "term_id": "GO:0006898",
  "gene_name": "Lysosome membrane protein 2",
  "gene": "UniProtKB:Q14108",
  "term_label": "receptor-mediated endocytosis"
}